{
  "term_label": "U5 snRNA binding",
  "gene_name": "Pre-mRNA-processing-splicing factor 8",
  "term_id": "GO:0030623",
  "gene_symbol": "PRPF8",
  "gene": "UniProtKB:Q6P2Q9"
}